{
  "gene_symbol": "IL23R",
  "gene_name": "Interleukin-23 receptor",
  "term_id": "GO:0042019",
  "gene": "UniProtKB:Q5VWK5",
  "term_label": "interleukin-23 binding"
}